{
  "gene_name": "Neuropeptide Y receptor type 4",
  "gene_symbol": "NPY4R",
  "term_label": "neuropeptide signaling pathway",
  "term_id": "GO:0007218",
  "gene": "UniProtKB:P50391"
}